{
  "term_id": "GO:0004527",
  "gene_symbol": "ISG20",
  "term_label": "exonuclease activity",
  "gene_name": "Interferon-stimulated gene 20 kDa protein",
  "gene": "UniProtKB:Q96AZ6"
}